{
  "term_id": "GO:0005634",
  "gene_symbol": "KIF18B",
  "gene": "UniProtKB:Q86Y91",
  "gene_name": "Kinesin-like protein KIF18B",
  "term_label": "nucleus"
}